positive regulation of calcineurin-mediated signaling [GO:0106058] (biological process) References: PMID:25081204 Relationships: is a type of GO:0050850; is_a regulation of calcineurin-mediated signaling [GO:0106056]; positively regulates calcineurin-mediated signaling [GO:0097720] Definition: Any process that activates or increases the frequency, rate or extent of calcineurin-mediated signaling. Subtypes: positive regulation of calcineurin-NFAT signaling cascade [GO:0070886]